{
  "term_id": "UNKNOWN:0001",
  "term_label": "Unknown molecular function",
  "gene_name": "Cancer_testis antigen family 45 member A7",
  "gene_symbol": "CT45A7",
  "gene": "UniProtKB:P0DMV0"
}